{
  "term_label": "Unknown cellular component",
  "gene_symbol": "LINC00052",
  "term_id": "UNKNOWN:0003",
  "gene_name": "Putative uncharacterized protein encoded by LINC00052",
  "gene": "UniProtKB:Q96N35"
}